hyphal septin cap [GO:0032164] (cellular component) Definition: A faint structure formed of septins found at the leading edge of growth in hyphae of fungal cells growing filamentously. This cap of septins colocalizes with a region of the plasma membrane that is rich in ergosterol. Relationships: is a type of septin cap [GO:0032159] References: PMID:16151244 Sources: GOC:krc